cholesterol oxidase activity [GO:0016995] (molecular function) Relationships: is a type of oxidoreductase activity, acting on the CH-OH group of donors, oxygen as acceptor [GO:0016899] Definition: Catalysis of the reaction: cholesterol + O2 = cholest-5-en-3-one + H2O2. Also known as: 3beta-hydroxy steroid oxidoreductase activity, 3beta-hydroxysteroid:oxygen oxidoreductase activity, cholesterol- O2 oxidoreductase activity, cholesterol-O2 oxidoreductase activity, cholesterol:oxygen oxidoreductase activity Sources: RHEA:32183